{
  "term_id": "GO:0016926",
  "gene_symbol": "SENP6",
  "term_label": "protein desumoylation",
  "gene": "UniProtKB:Q9GZR1",
  "gene_name": "Sentrin-specific protease 6"
}